canalicular bile acid transport [GO:0015722] (biological process) Definition: Enables the transfer of bile acid from one side of a hepatocyte plasma membrane into a bile canaliculus. Bile canaliculi are the thin tubes formed by hepatocyte membranes. Bile acids are any of a group of steroid carboxylic acids occurring in bile, where they are present as the sodium salts of their amides with glycine or taurine. Sources: GOC:dph Relationships: is a type of GO:0015721; is a type of secretion [GO:0046903]